{
  "gene_name": "Scavenger receptor class F member 2",
  "gene": "UniProtKB:Q96GP6",
  "gene_symbol": "SCARF2",
  "term_id": "GO:0005044",
  "term_label": "scavenger receptor activity"
}